{
  "gene": "UniProtKB:Q86VZ5",
  "gene_name": "Phosphatidylcholine:ceramide cholinephosphotransferase 1",
  "term_label": "ceramide biosynthetic process",
  "gene_symbol": "SGMS1",
  "term_id": "GO:0046513"
}